sulfite dehydrogenase activity [GO:0050310] (molecular function) Definition: Catalysis of the reaction: sulfite + 2 ferricytochrome c + H2O = sulfate + 2 ferrocytochrome c. Relationships: is a type of oxidoreductase activity, acting on a sulfur group of donors, cytochrome as acceptor [GO:0016669] Also known as: sulphite dehydrogenase activity, sulfite cytochrome c reductase activity, sulfite-cytochrome c oxidoreductase activity, sulfite:ferricytochrome-c oxidoreductase activity Sources: EC:1.8.2.1, MetaCyc:SULFITE-DEHYDROGENASE-RXN